apoptosome [GO:0043293] (cellular component) Definition: A multisubunit protein complex involved in the signaling phase of the apoptotic process. In mammals it is typically composed of seven Apaf-1 subunits bound to cytochrome c and caspase-9. A similar complex to promote apoptosis is formed from homologous gene products in other eukaryotic organisms. References: PMID:10428850, PMID:11406413, PMID:12176339, PMID:15189137 Sources: GOC:mtg_apoptosis Relationships: is a type of GO:0032991; is part of cytosol [GO:0005829]